{
  "gene": "UniProtKB:Q6PK57",
  "term_id": "UNKNOWN:0003",
  "gene_name": "Putative GED domain-containing protein DNM1P34",
  "term_label": "Unknown cellular component",
  "gene_symbol": "DNM1P34"
}